positive regulation of membrane invagination [GO:1905155] (BP) Relationships: is a type of positive regulation of cellular component organization [GO:0051130]; is a type of regulation of membrane invagination [GO:1905153]; positively regulates membrane invagination [GO:0010324] Also known as: up regulation of membrane invagination, up-regulation of membrane invagination, upregulation of membrane invagination, activation of membrane invagination Definition: Any process that activates or increases the frequency, rate or extent of membrane invagination. Sources: GOC:PARL, GOC:TermGenie, GOC:bf, GO_REF:0000058 Subtypes: positive regulation of phagocytosis, engulfment [GO:0060100]